cell cortex of growing cell tip [GO:1902716] (cellular component) References: PMID:24146635 Sources: GOC:TermGenie, GO_REF:0000064 Relationships: is a type of GO:0051285; BFO_0000050 growing cell tip [GO:0035838] Definition: Any cell cortex that is part of a growing cell tip. Also known as: cell cortex of growing cell end